{
  "term_id": "GO:0005886",
  "gene_name": "Proton channel OTOP1",
  "gene_symbol": "OTOP1",
  "term_label": "plasma membrane",
  "gene": "UniProtKB:Q7RTM1"
}